macrolide binding [GO:0005527] (molecular function) Definition: Binding to a macrolide, any of a large group of structurally related antibiotics produced by Streptomyces species. Subtypes: FK506 binding [GO:0005528], enterobactin binding [GO:1903981] Sources: GOC:jl, ISBN:0198506732 Relationships: is a type of binding [GO:0005488]